RNA 2',3'-cyclic 3'-phosphodiesterase activity [GO:0008664] (molecular function) Definition: Catalysis the reaction: a 3'-end 2',3'-cyclophospho-ribonucleotide-RNA + H2O = a 3'-end 2'-phospho-ribonucleotide-RNA + H+. Also known as: 2'-5' RNA ligase activity Relationships: is a type of phosphoric diester hydrolase activity [GO:0008081] References: PMID:25239919 Sources: RHEA:11828